{
  "gene_name": "G-protein coupled receptor 61",
  "gene": "UniProtKB:Q9BZJ8",
  "term_id": "GO:0004930",
  "term_label": "G protein-coupled receptor activity",
  "gene_symbol": "GPR61"
}